{
  "gene_name": "Golgi-associated kinase 1B",
  "term_label": "Unknown molecular function",
  "gene": "UniProtKB:Q6UWH4",
  "gene_symbol": "GASK1B",
  "term_id": "UNKNOWN:0001"
}